guanosine tetraphosphate biosynthetic process [GO:0015970] (biological process) Relationships: is_a purine ribonucleotide biosynthetic process [GO:0009152]; is a type of GO:0015969; is a type of GO:0034036 Also known as: guanosine tetraphosphate (5'-ppGpp-3') biosynthesis, guanosine tetraphosphate (5'-ppGpp-3') biosynthetic process, guanosine tetraphosphate anabolism, guanosine tetraphosphate biosynthesis, guanosine tetraphosphate formation, guanosine tetraphosphate synthesis Sources: GOC:ai Definition: The chemical reactions and pathways resulting in the formation of guanine tetraphosphate (5'-ppGpp-3'), a derivative of guanine riboside with four phosphates.